{
  "gene_symbol": "TCL1A",
  "term_id": "GO:0035556",
  "gene": "UniProtKB:P56279",
  "gene_name": "T-cell leukemia_lymphoma protein 1A",
  "term_label": "intracellular signal transduction"
}